{
  "gene_symbol": "PRR23E",
  "gene_name": "Proline-rich protein 23E",
  "gene": "UniProtKB:Q8N813",
  "term_label": "Unknown biological process",
  "term_id": "UNKNOWN:0002"
}